{
  "gene": "UniProtKB:Q7L5L3",
  "gene_symbol": "GDPD3",
  "gene_name": "Lysophospholipase D GDPD3",
  "term_id": "GO:0046475",
  "term_label": "glycerophospholipid catabolic process"
}